regulation of protein desumoylation [GO:0060188] (biological process) Definition: Any process that modulates the frequency, rate or extent of protein desumoylation. Protein desumoylation is the process in which a SUMO protein (small ubiquitin-related modifier) is cleaved from its target protein. Sources: GOC:dph, GOC:tb Relationships: is a type of regulation of protein modification by small protein conjugation or removal [GO:1903320]; regulates GO:0016926 Subtypes: positive regulation of protein desumoylation [GO:0060189], GO:0060190